mast cell secretory granule organization [GO:0033364] (biological process) Relationships: is a type of secretory granule organization [GO:0033363] Also known as: mast cell secretory granule organisation, mast cell secretory granule maturation, mast cell secretory granule organization and biogenesis Definition: A process that is carried out at the cellular level which results in the assembly, arrangement of constituent parts, or disassembly of a secretory granule in a mast cell. A secretory granule is a small subcellular vesicle, surrounded by a membrane, that is formed from the Golgi apparatus and contains a highly concentrated protein destined for secretion. Sources: GOC:mah